{
  "gene": "UniProtKB:Q9NSB2",
  "term_id": "GO:0031424",
  "gene_symbol": "KRT84",
  "gene_name": "Keratin, type II cuticular Hb4",
  "term_label": "keratinization"
}